{
  "term_label": "serine-type endopeptidase activity",
  "gene": "UniProtKB:Q8TEB9",
  "gene_name": "Rhomboid-related protein 4",
  "term_id": "GO:0004252",
  "gene_symbol": "RHBDD1"
}